{
  "gene_name": "Exocyst complex component 3-like protein 4",
  "term_id": "GO:0000145",
  "term_label": "exocyst",
  "gene_symbol": "EXOC3L4",
  "gene": "UniProtKB:Q17RC7"
}